plasmid recombination [GO:0042150] (biological process) Definition: A process of DNA recombination occurring within a plasmid or between plasmids and other plasmids or DNA molecules. Relationships: is a type of GO:0006310 Sources: GOC:mlg